{
  "gene_name": "Interleukin-20 receptor subunit beta",
  "term_id": "GO:0042015",
  "term_label": "interleukin-20 binding",
  "gene": "UniProtKB:Q6UXL0",
  "gene_symbol": "IL20RB"
}